{
  "term_label": "chromatin binding",
  "gene_symbol": "RING1",
  "gene_name": "E3 ubiquitin-protein ligase RING1",
  "gene": "UniProtKB:Q06587",
  "term_id": "GO:0003682"
}